{
  "gene": "UniProtKB:O95628",
  "gene_name": "CCR4-NOT transcription complex subunit 4",
  "gene_symbol": "CNOT4",
  "term_label": "ubiquitin-protein transferase activity",
  "term_id": "GO:0004842"
}